{
  "gene": "UniProtKB:Q8N614",
  "term_label": "Unknown cellular component",
  "gene_name": "Transmembrane protein 156",
  "term_id": "UNKNOWN:0003",
  "gene_symbol": "TMEM156"
}